{
  "gene": "UniProtKB:Q9NQI0",
  "term_label": "nucleus",
  "gene_name": "Probable ATP-dependent RNA helicase DDX4",
  "term_id": "GO:0005634",
  "gene_symbol": "DDX4"
}